{
  "gene": "UniProtKB:P40305",
  "term_id": "GO:0097193",
  "term_label": "intrinsic apoptotic signaling pathway",
  "gene_name": "Interferon alpha-inducible protein 27, mitochondrial",
  "gene_symbol": "IFI27"
}